regulation of cardioblast differentiation [GO:0051890] (biological process) Definition: Any process that modulates the frequency, rate or extent of cardioblast differentiation, the process in which a relatively unspecialized mesodermal cell acquires the specialized structural and/or functional features of a cardioblast. A cardioblast is a cardiac precursor cell. It is a cell that has been committed to a cardiac fate, but will undergo more cell division rather than terminally differentiating. Subtypes: regulation of cardioblast cell fate specification [GO:0042686], positive regulation of cardioblast differentiation [GO:0051891], negative regulation of cardioblast differentiation [GO:0051892], regulation of cardiac muscle cell myoblast differentiation [GO:2000690] Sources: GOC:ai Relationships: is a type of regulation of cardiocyte differentiation [GO:1905207]; is_a GO:2000736; regulates cardioblast differentiation [GO:0010002]